{
  "gene_symbol": "U2AF2",
  "gene": "UniProtKB:P26368",
  "term_label": "spliceosomal complex assembly",
  "gene_name": "Splicing factor U2AF 65 kDa subunit",
  "term_id": "GO:0000245"
}